{
  "gene": "UniProtKB:Q53GL7",
  "gene_symbol": "PARP10",
  "term_id": "GO:0003714",
  "gene_name": "Protein mono-ADP-ribosyltransferase PARP10",
  "term_label": "transcription corepressor activity"
}